{
  "term_id": "GO:0019731",
  "term_label": "antibacterial humoral response",
  "gene_symbol": "DEFA5",
  "gene": "UniProtKB:Q01523",
  "gene_name": "Defensin alpha 5"
}